{
  "gene_name": "SAYSvFN domain-containing protein 1",
  "gene": "UniProtKB:Q9NPB0",
  "term_label": "UFM1-modified protein reader activity",
  "term_id": "GO:0141185",
  "gene_symbol": "SAYSD1"
}